regulation of peripheral B cell deletion [GO:0002908] (biological process) Subtypes: negative regulation of peripheral B cell deletion [GO:0002909], positive regulation of peripheral B cell deletion [GO:0002910] Definition: Any process that modulates the frequency, rate, or extent of peripheral B cell deletion. Sources: GOC:add Relationships: is a type of regulation of peripheral tolerance induction [GO:0002658]; is a type of GO:0002712; is a type of regulation of B cell deletion [GO:0002867]; regulates peripheral B cell deletion [GO:0002454]